{
  "gene_symbol": "NDUFB10",
  "term_id": "GO:0045271",
  "term_label": "respiratory chain complex I",
  "gene": "UniProtKB:O96000",
  "gene_name": "NADH dehydrogenase [ubiquinone] 1 beta subcomplex subunit 10"
}